{
  "gene_symbol": "FAM187B",
  "term_label": "Unknown cellular component",
  "gene": "UniProtKB:Q17R55",
  "gene_name": "Protein FAM187B",
  "term_id": "UNKNOWN:0003"
}